{
  "term_label": "Unknown molecular function",
  "gene": "UniProtKB:Q14151",
  "gene_symbol": "SAFB2",
  "term_id": "UNKNOWN:0001",
  "gene_name": "Scaffold attachment factor B2"
}